pyrimidine deoxyribonucleoside triphosphate catabolic process [GO:0009213] (biological process) Also known as: pyrimidine deoxyribonucleoside triphosphate breakdown, pyrimidine deoxyribonucleoside triphosphate catabolism, pyrimidine deoxyribonucleoside triphosphate degradation Definition: The chemical reactions and pathways resulting in the breakdown of pyrimidine deoxyribonucleoside triphosphate, a compound consisting of a pyrimidine base linked to a deoxyribose sugar esterified with triphosphate on the sugar. Relationships: is a type of pyrimidine nucleoside triphosphate catabolic process [GO:0009149]; is a type of pyrimidine deoxyribonucleoside triphosphate metabolic process [GO:0009211] Sources: GOC:go_curators, ISBN:0198506732 Subtypes: dCTP catabolic process [GO:0006253], dTTP catabolic process [GO:0046076], dUTP catabolic process [GO:0046081]